{
  "gene_symbol": "NDUFA8",
  "gene": "UniProtKB:P51970",
  "term_label": "Unknown molecular function",
  "gene_name": "NADH dehydrogenase [ubiquinone] 1 alpha subcomplex subunit 8",
  "term_id": "UNKNOWN:0001"
}